{
  "term_label": "B cell receptor signaling pathway",
  "gene_symbol": "NFAM1",
  "gene_name": "NFAT activation molecule 1",
  "term_id": "GO:0050853",
  "gene": "UniProtKB:Q8NET5"
}